{
  "gene": "UniProtKB:P28069",
  "term_label": "DNA-binding transcription factor activity, RNA polymerase II-specific",
  "gene_name": "Pituitary-specific positive transcription factor 1",
  "gene_symbol": "POU1F1",
  "term_id": "GO:0000981"
}